{
  "term_label": "Unknown molecular function",
  "gene_name": "Keratin-associated protein 5-10",
  "term_id": "UNKNOWN:0001",
  "gene": "UniProtKB:Q6L8G5",
  "gene_symbol": "KRTAP5-10"
}